{
  "gene_symbol": "CCL21",
  "gene": "UniProtKB:O00585",
  "term_id": "GO:0048020",
  "gene_name": "C-C motif chemokine 21",
  "term_label": "CCR chemokine receptor binding"
}